{
  "term_id": "GO:0061589",
  "term_label": "calcium activated phosphatidylserine scrambling",
  "gene": "UniProtKB:A1A5B4",
  "gene_symbol": "ANO9",
  "gene_name": "Anoctamin-9"
}